{
  "gene_symbol": "SLC22A31",
  "gene": "UniProtKB:A6NKX4",
  "gene_name": "Putative solute carrier family 22 member 31",
  "term_label": "Unknown molecular function",
  "term_id": "UNKNOWN:0001"
}